{
  "gene_symbol": "DARS1",
  "term_label": "aminoacyl-tRNA synthetase multienzyme complex",
  "gene_name": "Aspartate--tRNA ligase, cytoplasmic",
  "term_id": "GO:0017101",
  "gene": "UniProtKB:P14868"
}